{
  "gene_symbol": "GSTT2B",
  "gene_name": "Glutathione S-transferase theta-2B",
  "gene": "UniProtKB:P0CG30",
  "term_id": "GO:0004364",
  "term_label": "glutathione transferase activity"
}